floor plate formation [GO:0021508] (biological process) Definition: The formation of a ventral region of glial cells in the neural tube that provides inductive signals for the specification of neuronal cell types. The floor plate is evident at the ventral midline by the neural fold stage. References: PMID:11262869 Sources: GOC:cls, GOC:dgh, GOC:dph, GOC:jid, GO_REF:0000021 Relationships: is a type of anatomical structure formation involved in morphogenesis [GO:0048646]; is part of ventral midline development [GO:0007418]; is part of floor plate morphogenesis [GO:0033505]